{
  "gene": "UniProtKB:Q13596",
  "term_label": "endosome membrane",
  "term_id": "GO:0010008",
  "gene_symbol": "SNX1",
  "gene_name": "Sorting nexin-1"
}